rubredoxin-NAD+ reductase activity [GO:0015044] (molecular function) Definition: Catalysis of the reaction: 2 reduced [rubredoxin] + NAD+ + H+ = 2 oxidized [rubredoxin] + NADH. Sources: RHEA:18597 Also known as: NADH:rubredoxin reductase activity, DPNH-rubredoxin reductase activity, NADH--rubredoxin oxidoreductase activity, NADH--rubredoxin reductase activity, NADH:rubredoxin oxidoreductase activity, dihydronicotinamide adenine dinucleotide--rubredoxin reductase activity, reduced nicotinamide adenine dinucleotide--rubredoxin reductase activity, rubredoxin--NAD reductase activity, rubredoxin--nicotinamide adenine dinucleotide reductase activity, rubredoxin:NAD+ oxidoreductase activity Relationships: is a type of rubredoxin-NAD(P)H reductase activity [GO:0015045]